{
  "gene_symbol": "CRPPA",
  "gene": "UniProtKB:A4D126",
  "term_label": "protein O-linked glycosylation via mannose",
  "term_id": "GO:0035269",
  "gene_name": "D-ribitol-5-phosphate cytidylyltransferase"
}